{
  "gene_symbol": "POFUT2",
  "term_label": "Unknown biological process",
  "gene": "UniProtKB:Q9Y2G5",
  "term_id": "UNKNOWN:0002",
  "gene_name": "GDP-fucose protein O-fucosyltransferase 2"
}